{
  "gene": "UniProtKB:Q969V6",
  "gene_symbol": "MRTFA",
  "gene_name": "Myocardin-related transcription factor A",
  "term_label": "nucleus",
  "term_id": "GO:0005634"
}